endocannabinoid signaling pathway involved in retrograde trans-synaptic signaling [GO:1905197] (biological process) References: PMID:23040807 Sources: GOC:TermGenie, GO_REF:0000060 Relationships: is a type of GO:1905129; is part of retrograde trans-synaptic signaling by endocannabinoid [GO:0098921] Definition: Any endocannabinoid signaling pathway that is involved in retrograde trans-synaptic signaling by endocannabinoid. Also known as: endocannabinoid signalling pathway involved in retrograde trans-synaptic signaling by endocannabinoid